wing disc pattern formation [GO:0035222] (biological process) Relationships: is a type of imaginal disc pattern formation [GO:0007447]; is part of GO:0035220 Definition: The process giving rise to the pattern of cell differentiation in the wing imaginal disc. Subtypes: wing disc proximal/distal pattern formation [GO:0007473], wing disc anterior/posterior pattern formation [GO:0048100], wing disc dorsal/ventral pattern formation [GO:0048190] Sources: GOC:bf